{
  "term_id": "GO:0016192",
  "gene_name": "Ras-related protein Rab-39B",
  "term_label": "vesicle-mediated transport",
  "gene_symbol": "RAB39B",
  "gene": "UniProtKB:Q96DA2"
}